{
  "gene": "UniProtKB:Q15269",
  "term_label": "small-subunit processome",
  "term_id": "GO:0032040",
  "gene_symbol": "PWP2",
  "gene_name": "Periodic tryptophan protein 2 homolog"
}